{
  "gene": "UniProtKB:Q14088",
  "term_id": "GO:0003924",
  "term_label": "GTPase activity",
  "gene_symbol": "RAB33A",
  "gene_name": "Ras-related protein Rab-33A"
}